{
  "gene_name": "POU domain, class 5, transcription factor 2",
  "gene": "UniProtKB:Q8N7G0",
  "term_label": "DNA-binding transcription factor activity, RNA polymerase II-specific",
  "gene_symbol": "POU5F2",
  "term_id": "GO:0000981"
}